{
  "gene_symbol": "HACE1",
  "gene": "UniProtKB:Q8IYU2",
  "term_label": "ubiquitin protein ligase activity",
  "gene_name": "E3 ubiquitin-protein ligase HACE1",
  "term_id": "GO:0061630"
}